{
  "gene_symbol": "XPC",
  "term_id": "GO:0000111",
  "gene_name": "DNA repair protein complementing XP-C cells",
  "gene": "UniProtKB:Q01831",
  "term_label": "nucleotide-excision repair factor 2 complex"
}